{
  "gene_symbol": "UCHL5",
  "gene": "UniProtKB:Q9Y5K5",
  "gene_name": "Ubiquitin carboxyl-terminal hydrolase isozyme L5",
  "term_label": "regulation of chromosome organization",
  "term_id": "GO:0033044"
}